{
  "gene_name": "GPI ethanolamine phosphate transferase 1",
  "term_id": "GO:0005789",
  "term_label": "endoplasmic reticulum membrane",
  "gene_symbol": "PIGN",
  "gene": "UniProtKB:O95427"
}